spleen development [GO:0048536] (biological process) Definition: The process whose specific outcome is the progression of the spleen over time, from its formation to the mature structure. The spleen is a large vascular lymphatic organ composed of white and red pulp, involved both in hemopoietic and immune system functions. Sources: GOC:add, ISBN:0781735149 Relationships: is a type of hematopoietic or lymphoid organ development [GO:0048534]